{
  "term_id": "GO:0051603",
  "gene_symbol": "CTSS",
  "gene": "UniProtKB:P25774",
  "gene_name": "Cathepsin S",
  "term_label": "proteolysis involved in protein catabolic process"
}